{
  "gene": "UniProtKB:Q6DRA6",
  "gene_symbol": "H2BC19P",
  "term_id": "GO:0000786",
  "term_label": "nucleosome",
  "gene_name": "Putative histone H2B type 2-D"
}